half bridge of mitotic spindle pole body [GO:0061496] (cellular component) Definition: Structure adjacent to the plaques of the mitotic spindle pole body. Relationships: is_a GO:0005825; is part of mitotic spindle pole body [GO:0044732] Sources: GOC:dph